{
  "term_label": "Unknown cellular component",
  "gene": "UniProtKB:P20333",
  "term_id": "UNKNOWN:0003",
  "gene_name": "Tumor necrosis factor receptor superfamily member 1B",
  "gene_symbol": "TNFRSF1B"
}